endoplasmic reticulum tubular network membrane [GO:0098826] (CC) Definition: The membrane of the endoplasmic reticulum tubular network. References: PMID:16469703 Relationships: is a type of endoplasmic reticulum membrane [GO:0005789]; is part of GO:0071782 Subtypes: cortical endoplasmic reticulum membrane [GO:0160219]